{
  "gene_name": "Biotinidase",
  "term_id": "UNKNOWN:0001",
  "gene": "UniProtKB:P43251",
  "gene_symbol": "BTD",
  "term_label": "Unknown molecular function"
}